ErbB-2 class receptor binding [GO:0005176] (molecular function) Definition: Binding to a protein-tyrosine kinase receptor Neu/ErbB-2/HER2. Sources: GOC:jl Also known as: HER2 receptor binding, Neu receptor binding, ErbB-2 class receptor ligand, HER2 receptor ligand, Neu receptor ligand Relationships: is a type of signaling receptor binding [GO:0005102]